2-dehydro-3-deoxy-D-gluconic acid catabolic process [GO:1901273] (biological process) Sources: GOC:TermGenie, GOC:yaf, UniPathway:UPA00856 Relationships: is_a monosaccharide catabolic process [GO:0046365]; is a type of monocarboxylic acid catabolic process [GO:0072329] Definition: The chemical reactions and pathways resulting in the breakdown of 2-dehydro-3-deoxy-D-gluconic acid. Also known as: 2-dehydro-3-deoxy-D-gluconic acid breakdown, 2-dehydro-3-deoxy-D-gluconic acid catabolism, 2-dehydro-3-deoxy-D-gluconic acid degradation